{
  "term_id": "GO:0005943",
  "term_label": "phosphatidylinositol 3-kinase complex, class IA",
  "gene_name": "Phosphatidylinositol 3-kinase regulatory subunit gamma",
  "gene": "UniProtKB:Q92569",
  "gene_symbol": "PIK3R3"
}